{
  "term_id": "GO:0031932",
  "term_label": "TORC2 complex",
  "gene_symbol": "MAPKAP1",
  "gene": "UniProtKB:Q9BPZ7",
  "gene_name": "Target of rapamycin complex 2 subunit MAPKAP1"
}